{
  "gene_name": "Coatomer subunit beta'",
  "gene": "UniProtKB:P35606",
  "term_id": "UNKNOWN:0001",
  "gene_symbol": "COPB2",
  "term_label": "Unknown molecular function"
}